{
  "gene": "UniProtKB:Q8N720",
  "term_label": "nucleus",
  "gene_symbol": "ZNF655",
  "gene_name": "Zinc finger protein 655",
  "term_id": "GO:0005634"
}